{
  "term_id": "GO:0005739",
  "term_label": "mitochondrion",
  "gene_symbol": "TACO1",
  "gene": "UniProtKB:Q9BSH4",
  "gene_name": "Translational activator of cytochrome c oxidase 1"
}